eukaryotic elongation factor-2 kinase activator activity [GO:0042557] (molecular function) Also known as: eEF-2 kinase activator References: PMID:11904175 Sources: GOC:jl Relationships: is a type of eukaryotic elongation factor-2 kinase regulator activity [GO:0042556]; is_a GO:0043539; positively regulates elongation factor-2 kinase activity [GO:0004686] Definition: Binds to and increases the activity of the enzyme eukaryotic elongation factor-2 kinase.